positive regulation of tRNA methylation [GO:0110004] (biological process) References: PMID:23074192 Sources: GOC:vw Definition: Any process that activates or increases the frequency, rate or extent of tRNA methylation. Subtypes: positive regulation of tRNA C5-cytosine methylation [GO:0110005] Relationships: is a type of regulation of tRNA methylation [GO:0110002]; is a type of positive regulation of tRNA processing [GO:2000237]; positively regulates GO:0030488